{
  "gene_symbol": "ZNF487",
  "term_id": "GO:0000981",
  "gene": "UniProtKB:B1APH4",
  "gene_name": "Putative zinc finger protein 487",
  "term_label": "DNA-binding transcription factor activity, RNA polymerase II-specific"
}